replication compartment [GO:0046809] (cellular component) Relationships: is a type of nuclear viral factory [GO:0039715] Definition: Globular nuclear domains where the transcription and replication of the viral genome occurs. More than one site can be present simultaneously. References: PMID:9499108 Sources: VZ:1951 Also known as: RC